{
  "gene_name": "Ubiquitin carboxyl-terminal hydrolase 37",
  "gene": "UniProtKB:Q86T82",
  "gene_symbol": "USP37",
  "term_label": "nucleus",
  "term_id": "GO:0005634"
}